dihydroneopterin aldolase activity [GO:0004150] (molecular function) Definition: Catalysis of the reaction: 2-amino-4-hydroxy-6-(D-erythro-1,2,3-trihydroxypropyl)-7,8-dihydropteridine = 2-amino-4-hydroxy-6-hydroxymethyl-7,8-dihydropteridine + glycolaldehyde. Sources: EC:4.1.2.25 Relationships: is a type of GO:0016832 Also known as: 2-amino-4-hydroxy-6-(D-erythro-1,2,3-trihydroxypropyl)-7,8-dihydropteridine glycolaldehyde-lyase (2-amino-4-hydroxy-6-hydroxymethyl-7,8-dihydropteridine-forming), 2-amino-4-hydroxy-6-(D-erythro-1,2,3-trihydroxypropyl)-7,8-dihydropteridine glycolaldehyde-lyase activity